{
  "term_id": "GO:0030280",
  "gene": "UniProtKB:O76015",
  "gene_symbol": "KRT38",
  "term_label": "structural constituent of skin epidermis",
  "gene_name": "Keratin, type I cuticular Ha8"
}